{
  "term_label": "cell surface receptor signaling pathway",
  "gene_symbol": "FCGR3A",
  "gene": "UniProtKB:P08637",
  "term_id": "GO:0007166",
  "gene_name": "Low affinity immunoglobulin gamma Fc region receptor III-A"
}